{
  "term_label": "RNA polymerase II cis-regulatory region sequence-specific DNA binding",
  "term_id": "GO:0000978",
  "gene_symbol": "ZNF727",
  "gene": "UniProtKB:A8MUV8",
  "gene_name": "Putative zinc finger protein 727"
}